{
  "gene_symbol": "SMARCD1",
  "gene_name": "SWI_SNF-related matrix-associated actin-dependent regulator of chromatin subfamily D member 1",
  "term_label": "nucleus",
  "gene": "UniProtKB:Q96GM5",
  "term_id": "GO:0005634"
}